smooth septate junction [GO:0005920] (cellular component) References: PMID:11700298 Also known as: zonula continua Relationships: is a type of septate junction [GO:0005918] Definition: A septate junction that lacks the regular arrays of electron-dense septae found in pleated septate junctions.